{
  "gene": "UniProtKB:Q9H1K4",
  "term_id": "GO:0043490",
  "gene_name": "Mitochondrial glutamate carrier 2",
  "term_label": "malate-aspartate shuttle",
  "gene_symbol": "SLC25A18"
}